{
  "gene": "UniProtKB:Q7RTU7",
  "term_id": "GO:0000977",
  "gene_name": "Basic helix-loop-helix transcription factor scleraxis",
  "gene_symbol": "SCX",
  "term_label": "RNA polymerase II transcription regulatory region sequence-specific DNA binding"
}